{
  "gene_symbol": "SWI5",
  "gene": "UniProtKB:Q1ZZU3",
  "gene_name": "DNA repair protein SWI5 homolog",
  "term_label": "double-strand break repair via homologous recombination",
  "term_id": "GO:0000724"
}